{
  "term_id": "UNKNOWN:0001",
  "term_label": "Unknown molecular function",
  "gene": "UniProtKB:Q5SWH9",
  "gene_name": "Transmembrane protein 69",
  "gene_symbol": "TMEM69"
}